{
  "term_id": "UNKNOWN:0003",
  "gene_symbol": "PKHD1L1",
  "gene": "UniProtKB:Q86WI1",
  "term_label": "Unknown cellular component",
  "gene_name": "Fibrocystin-L"
}